{
  "gene": "UniProtKB:Q5T5Y3",
  "gene_name": "Calmodulin-regulated spectrin-associated protein 1",
  "gene_symbol": "CAMSAP1",
  "term_label": "Unknown cellular component",
  "term_id": "UNKNOWN:0003"
}